{
  "gene": "UniProtKB:P83436",
  "gene_name": "Conserved oligomeric Golgi complex subunit 7",
  "term_id": "GO:0017119",
  "term_label": "Golgi transport complex",
  "gene_symbol": "COG7"
}